{
  "gene": "UniProtKB:P30939",
  "term_label": "dendrite",
  "term_id": "GO:0030425",
  "gene_symbol": "HTR1F",
  "gene_name": "5-hydroxytryptamine receptor 1F"
}